{
  "term_label": "cytosolic [4Fe-4S] assembly targeting complex",
  "gene_name": "Cytosolic iron-sulfur assembly component 3",
  "gene": "UniProtKB:Q9H6Q4",
  "term_id": "GO:0097361",
  "gene_symbol": "CIAO3"
}